{
  "term_id": "GO:0005681",
  "term_label": "spliceosomal complex",
  "gene_name": "Thioredoxin-like protein 4A",
  "gene": "UniProtKB:P83876",
  "gene_symbol": "TXNL4A"
}